{
  "term_id": "GO:0051960",
  "gene_symbol": "GBX2",
  "term_label": "regulation of nervous system development",
  "gene": "UniProtKB:P52951",
  "gene_name": "Homeobox protein GBX-2"
}